{
  "gene_name": "UDP-glucuronosyltransferase 2A2",
  "term_label": "Unknown biological process",
  "gene_symbol": "UGT2A2",
  "gene": "UniProtKB:P0DTE5",
  "term_id": "UNKNOWN:0002"
}